{
  "term_label": "juxtaparanode region of axon",
  "term_id": "GO:0044224",
  "gene": "UniProtKB:Q09470",
  "gene_symbol": "KCNA1",
  "gene_name": "Potassium voltage-gated channel subfamily A member 1"
}